{
  "term_label": "cytoplasm",
  "gene": "UniProtKB:Q8IYT8",
  "term_id": "GO:0005737",
  "gene_symbol": "ULK2",
  "gene_name": "Serine_threonine-protein kinase ULK2"
}